{
  "gene_name": "Monofunctional C1-tetrahydrofolate synthase, mitochondrial",
  "term_id": "GO:0009257",
  "gene": "UniProtKB:Q6UB35",
  "gene_symbol": "MTHFD1L",
  "term_label": "10-formyltetrahydrofolate biosynthetic process"
}